{
  "term_label": "cytoplasm",
  "term_id": "GO:0005737",
  "gene": "UniProtKB:Q6NZY7",
  "gene_name": "Cdc42 effector protein 5",
  "gene_symbol": "CDC42EP5"
}